{
  "gene_symbol": "KCNN2",
  "term_id": "GO:0071805",
  "term_label": "potassium ion transmembrane transport",
  "gene_name": "Small conductance calcium-activated potassium channel protein 2",
  "gene": "UniProtKB:Q9H2S1"
}